{
  "gene": "UniProtKB:Q15915",
  "gene_symbol": "ZIC1",
  "term_label": "central nervous system development",
  "term_id": "GO:0007417",
  "gene_name": "Zinc finger protein ZIC 1"
}